{
  "gene": "UniProtKB:Q96HR3",
  "term_label": "positive regulation of DNA-templated transcription",
  "term_id": "GO:0045893",
  "gene_symbol": "MED30",
  "gene_name": "Mediator of RNA polymerase II transcription subunit 30"
}